{
  "term_id": "GO:0003351",
  "term_label": "epithelial cilium movement involved in extracellular fluid movement",
  "gene_symbol": "DNAAF2",
  "gene_name": "Protein kintoun",
  "gene": "UniProtKB:Q9NVR5"
}